pyrokinin receptor activity [GO:0036401] (molecular function) Definition: Combining with a pyrokinin and transmitting the signal within the cell to induce a change in cell activity. Pyrokinins are a group of insect neuropeptides that share the common C-terminal pentapeptide sequence Phe-X-Pro-Arg-Leu-NH2 (X = S, T, K, A, or G). They play a central role in diverse physiological processes including stimulation of gut motility, production and release of sex pheromones, diapause, and pupariation. Relationships: is a type of neuropeptide receptor activity [GO:0008188] Also known as: PK receptor activity References: PMID:12951076, PMID:19186060 Sources: GOC:ha